{
  "term_label": "immunoglobulin mediated immune response",
  "gene_symbol": "IGHV2OR16-5",
  "term_id": "GO:0016064",
  "gene_name": "Immunoglobulin heavy variable 2_OR16-5 (non-functional) (Fragment)",
  "gene": "UniProtKB:A0A0B4J2B6"
}